{
  "term_id": "GO:0007157",
  "gene_name": "Pregnancy-specific beta-1-glycoprotein 5",
  "gene_symbol": "PSG5",
  "gene": "UniProtKB:Q15238",
  "term_label": "heterophilic cell-cell adhesion"
}